{
  "term_id": "GO:0008525",
  "gene_name": "Membrane-associated phosphatidylinositol transfer protein 2",
  "gene_symbol": "PITPNM2",
  "gene": "UniProtKB:Q9BZ72",
  "term_label": "phosphatidylcholine transporter activity"
}